{
  "gene_name": "Alpha-1D adrenergic receptor",
  "term_label": "plasma membrane",
  "gene": "UniProtKB:P25100",
  "gene_symbol": "ADRA1D",
  "term_id": "GO:0005886"
}